ligase activity, forming nitrogen-metal bonds, forming coordination complexes [GO:0051003] (molecular function) Relationships: is_a GO:0051002 Sources: EC:6.6.1.- Subtypes: magnesium chelatase activity [GO:0016851], cobaltochelatase activity [GO:0051116] Definition: Catalysis of the ligation of two substances via a nitrogen-metal bond, forming a coordination complex.